{
  "gene_name": "Growth arrest and DNA damage-inducible protein GADD45 alpha",
  "gene_symbol": "GADD45A",
  "gene": "UniProtKB:P24522",
  "term_id": "GO:0005737",
  "term_label": "cytoplasm"
}